{
  "gene_name": "Neurocan core protein",
  "term_id": "GO:0005615",
  "gene_symbol": "NCAN",
  "gene": "UniProtKB:O14594",
  "term_label": "extracellular space"
}